sphingomyelin biosynthetic process [GO:0006686] (biological process) Relationships: is a type of sphingomyelin metabolic process [GO:0006684]; is a type of phospholipid biosynthetic process [GO:0008654]; is a type of sphingolipid biosynthetic process [GO:0030148]; is a type of amide biosynthetic process [GO:0043604] Also known as: sphingomyelin anabolism, sphingomyelin biosynthesis, sphingomyelin formation, sphingomyelin synthesis Sources: ISBN:0198506732 Definition: The chemical reactions and pathways resulting in the formation of sphingomyelin, N-acyl-4-sphingenyl-1-O-phosphorylcholine.